{
  "gene": "UniProtKB:P54619",
  "gene_name": "5'-AMP-activated protein kinase subunit gamma-1",
  "gene_symbol": "PRKAG1",
  "term_id": "GO:0042149",
  "term_label": "cellular response to glucose starvation"
}